{
  "term_id": "GO:0098693",
  "gene_name": "DnaJ homolog subfamily C member 5",
  "gene_symbol": "DNAJC5",
  "term_label": "regulation of synaptic vesicle cycle",
  "gene": "UniProtKB:Q9H3Z4"
}